phosphatidylserine metabolic process [GO:0006658] (biological process) Also known as: phosphatidylserine metabolism Definition: The chemical reactions and pathways involving phosphatidylserines, any of a class of glycerophospholipids in which the phosphatidyl group is esterified to the hydroxyl group of L-serine. They are important constituents of cell membranes. Relationships: is a type of modified amino acid metabolic process [GO:0006575]; is a type of glycerophospholipid metabolic process [GO:0006650] Sources: ISBN:0198506732 Subtypes: phosphatidylserine biosynthetic process [GO:0006659], GO:0006660, phosphatidylserine acyl-chain remodeling [GO:0036150]